{
  "term_id": "GO:0007155",
  "gene_symbol": "PCDHB3",
  "term_label": "cell adhesion",
  "gene": "UniProtKB:Q9Y5E6",
  "gene_name": "Protocadherin beta-3"
}